{
  "term_label": "antigen processing and presentation of exogenous peptide antigen via MHC class II",
  "gene": "UniProtKB:P01903",
  "gene_symbol": "HLA-DRA",
  "gene_name": "HLA class II histocompatibility antigen, DR alpha chain",
  "term_id": "GO:0019886"
}